{
  "gene_symbol": "TDRD9",
  "term_id": "GO:0005634",
  "gene_name": "ATP-dependent RNA helicase TDRD9",
  "term_label": "nucleus",
  "gene": "UniProtKB:Q8NDG6"
}